ensheathment of neuronal cell bodies [GO:0032295] (biological process) Definition: The process in which satellite glial cells isolate neuronal cell bodies. Sources: GOC:dgh Relationships: is a type of ensheathment of neurons [GO:0007272]